{
  "gene_name": "Claudin-14",
  "term_label": "plasma membrane",
  "gene_symbol": "CLDN14",
  "gene": "UniProtKB:O95500",
  "term_id": "GO:0005886"
}